cellular response to lead ion [GO:0071284] (biological process) Sources: GOC:mah Relationships: is a type of GO:0010288; is a type of cellular response to metal ion [GO:0071248] Definition: Any process that results in a change in state or activity of a cell (in terms of movement, secretion, enzyme production, gene expression, etc.) as a result of a lead ion stimulus.